{
  "gene_symbol": "MKKS",
  "gene": "UniProtKB:Q9NPJ1",
  "gene_name": "Molecular chaperone MKKS",
  "term_id": "GO:0060271",
  "term_label": "cilium assembly"
}